subpallium radially oriented migration [GO:0021981] (biological process) Sources: GOC:cls, GOC:dgh, GOC:dph, GOC:jid, GO_REF:0000021 Definition: The migration of cells in the developing subpallium in which cells move from the ventricular and/or subventricular zone toward the surface of the brain. Relationships: is_a subpallium cell migration [GO:0021980]